{
  "gene": "UniProtKB:Q14457",
  "gene_symbol": "BECN1",
  "term_label": "phagophore assembly site",
  "term_id": "GO:0000407",
  "gene_name": "Beclin-1"
}